{
  "term_id": "GO:0005634",
  "term_label": "nucleus",
  "gene": "UniProtKB:A6NNM3",
  "gene_symbol": "RIMBP3B",
  "gene_name": "RIMS-binding protein 3B"
}